{
  "gene_name": "Metalloprotease TIKI2",
  "gene_symbol": "TRABD2B",
  "term_label": "negative regulation of Wnt signaling pathway",
  "gene": "UniProtKB:A6NFA1",
  "term_id": "GO:0030178"
}